{
  "gene_symbol": "HIRA",
  "gene_name": "Protein HIRA",
  "term_label": "chromatin remodeling",
  "term_id": "GO:0006338",
  "gene": "UniProtKB:P54198"
}